negative regulation of adenylate cyclase-activating glucose-activated G protein-coupled receptor signaling pathway [GO:0110034] (biological process) References: PMID:24297439 Sources: GOC:al Also known as: negative regulation of adenylate cyclase-activating glucose-activated G-protein coupled receptor signaling pathway Relationships: is a type of negative regulation of adenylate cyclase-activating G protein-coupled receptor signaling pathway [GO:0106072]; is a type of regulation of adenylate cyclase-activating glucose-activated G protein-coupled receptor signaling pathway [GO:0110033]; is a type of negative regulation of glucose mediated signaling pathway [GO:1902660]; negatively regulates adenylate cyclase-activating glucose-activated G protein-coupled receptor signaling pathway [GO:0010619] Definition: Any process that stops, prevents, or reduces the frequency, rate or extent of the adenylate cyclase-activating glucose-activated G protein-coupled receptor signaling pathway.